stem cell differentiation [GO:0048863] (biological process) Relationships: is a type of cell differentiation [GO:0030154] Definition: The process in which a relatively unspecialized cell acquires specialized features of a stem cell. A stem cell is a cell that retains the ability to divide and proliferate throughout life to provide progenitor cells that can differentiate into specialized cells. Subtypes: GO:0010002, neural crest cell differentiation [GO:0014033], GO:0035779, GO:0060218, squamous basal epithelial stem cell differentiation involved in prostate gland acinus development [GO:0060529], limb basal epidermal cell differentiation [GO:0060889], hepatoblast differentiation [GO:0061017], mesenchymal stem cell differentiation [GO:0072497], GO:1902691 Sources: CL:0000034, GOC:isa_complete Regulation: regulated by regulation of stem cell differentiation [GO:2000736]; negatively regulated by GO:2000737; positively regulated by GO:2000738